DNA replication checkpoint signaling [GO:0000076] (biological process) References: PMID:11728327, PMID:12537518 Sources: GOC:curators, GOC:rn Relationships: is a type of DNA integrity checkpoint signaling [GO:0031570] Subtypes: mitotic DNA replication checkpoint signaling [GO:0033314], GO:0033315 Definition: A signal transduction process that contributes to a DNA replication checkpoint, that prevents the initiation of nuclear division until DNA replication is complete, thereby ensuring that progeny inherit a full complement of the genome. Also known as: DNA replication checkpoint, signal transduction involved in DNA replication checkpoint